negative regulation of protein localization to chromosome, telomeric region [GO:1904815] (biological process) Definition: Any process that stops, prevents or reduces the frequency, rate or extent of protein localization to chromosome, telomeric region. References: PMID:19487455 Sources: GOC:BHF, GOC:BHF_telomere, GOC:TermGenie, GOC:nc, GO_REF:0000058 Relationships: is a type of GO:1903828; is a type of regulation of protein localization to chromosome, telomeric region [GO:1904814]; negatively regulates GO:0070198 Also known as: down regulation of protein localisation to chromosome, telomeric region, down regulation of protein localization to chromosome, telomeric region, down regulation of protein localization to telomere, down-regulation of protein localisation to chromosome, telomeric region, down-regulation of protein localization to chromosome, telomeric region, down-regulation of protein localization to telomere, downregulation of protein localisation to chromosome, telomeric region, downregulation of protein localization to chromosome, telomeric region, downregulation of protein localization to telomere, negative regulation of protein localisation to chromosome, telomeric region, negative regulation of protein localization to telomere, inhibition of protein localisation to chromosome, telomeric region, inhibition of protein localization to chromosome, telomeric region, inhibition of protein localization to telomere